cAMP response element binding protein binding [GO:0008140] (molecular function) Sources: GOC:mah Definition: Binding to a cAMP response element binding protein (a CREB protein). Also known as: 3',5' cAMP response element binding protein binding, 3',5'-cAMP response element binding protein binding, CREB binding, adenosine 3',5'-cyclophosphate response element binding protein binding, cyclic AMP response element binding protein binding, CBP Relationships: is a type of DNA-binding transcription factor binding [GO:0140297]